{
  "term_label": "cell surface",
  "gene_symbol": "CLEC9A",
  "gene_name": "C-type lectin domain family 9 member A",
  "gene": "UniProtKB:Q6UXN8",
  "term_id": "GO:0009986"
}